{
  "gene_name": "Protein S100-A16",
  "term_label": "nucleus",
  "gene": "UniProtKB:Q96FQ6",
  "term_id": "GO:0005634",
  "gene_symbol": "S100A16"
}